{
  "term_label": "negative regulation of transcription by RNA polymerase II",
  "gene": "UniProtKB:Q9Y3T9",
  "gene_symbol": "NOC2L",
  "gene_name": "Nucleolar complex protein 2 homolog",
  "term_id": "GO:0000122"
}